{
  "gene_name": "Argininosuccinate synthase",
  "gene_symbol": "ASS1",
  "term_id": "GO:0000050",
  "gene": "UniProtKB:P00966",
  "term_label": "urea cycle"
}